{
  "gene_symbol": "TGFBR3L",
  "gene": "UniProtKB:H3BV60",
  "term_id": "GO:0007179",
  "term_label": "transforming growth factor beta receptor signaling pathway",
  "gene_name": "Transforming growth factor-beta receptor type 3-like protein"
}